{
  "gene_name": "Embigin",
  "term_id": "GO:0070593",
  "gene": "UniProtKB:Q6PCB8",
  "term_label": "dendrite self-avoidance",
  "gene_symbol": "EMB"
}